negative regulation of synoviocyte proliferation [GO:1901646] (biological process) Sources: GOC:TermGenie Relationships: is_a GO:0050680; is a type of GO:1901645; negatively regulates GO:0002941 Definition: Any process that stops, prevents or reduces the frequency, rate or extent of synoviocyte proliferation. Also known as: down regulation of synoviocyte proliferation, down-regulation of synoviocyte proliferation, downregulation of synoviocyte proliferation, inhibition of synoviocyte proliferation